{
  "term_label": "protein import into peroxisome matrix, docking",
  "term_id": "GO:0016560",
  "gene": "UniProtKB:Q8IYB4",
  "gene_symbol": "PEX5L",
  "gene_name": "PEX5-related protein"
}